{
  "gene": "UniProtKB:P17023",
  "gene_name": "Zinc finger protein 19",
  "term_label": "nucleus",
  "term_id": "GO:0005634",
  "gene_symbol": "ZNF19"
}